{
  "term_id": "GO:0005737",
  "term_label": "cytoplasm",
  "gene_symbol": "HDAC9",
  "gene_name": "Histone deacetylase 9",
  "gene": "UniProtKB:Q9UKV0"
}